{
  "gene_symbol": "PI16",
  "gene": "UniProtKB:Q6UXB8",
  "gene_name": "Peptidase inhibitor 16",
  "term_id": "GO:0005615",
  "term_label": "extracellular space"
}